{
  "gene_symbol": "THBD",
  "term_label": "Unknown cellular component",
  "gene_name": "Thrombomodulin",
  "gene": "UniProtKB:P07204",
  "term_id": "UNKNOWN:0003"
}